{
  "gene_name": "Cholinesterase",
  "term_label": "plasma membrane",
  "gene": "UniProtKB:P06276",
  "term_id": "GO:0005886",
  "gene_symbol": "BCHE"
}